{
  "term_id": "GO:0042796",
  "gene_name": "Little elongation complex subunit 1",
  "gene": "UniProtKB:Q9Y2F5",
  "term_label": "snRNA transcription by RNA polymerase III",
  "gene_symbol": "ICE1"
}